{
  "term_label": "Unknown molecular function",
  "gene": "UniProtKB:Q96AN5",
  "gene_name": "Transmembrane protein 143",
  "gene_symbol": "TMEM143",
  "term_id": "UNKNOWN:0001"
}